{
  "term_label": "cytosol",
  "term_id": "GO:0005829",
  "gene_symbol": "USP34",
  "gene": "UniProtKB:Q70CQ2",
  "gene_name": "Ubiquitin carboxyl-terminal hydrolase 34"
}